{
  "gene_symbol": "TMCO2",
  "gene": "UniProtKB:Q7Z6W1",
  "term_id": "UNKNOWN:0001",
  "term_label": "Unknown molecular function",
  "gene_name": "Transmembrane and coiled-coil domain-containing protein 2"
}